{
  "term_label": "plasma membrane",
  "gene_name": "Olfactory receptor 51B4",
  "term_id": "GO:0005886",
  "gene": "UniProtKB:Q9Y5P0",
  "gene_symbol": "OR51B4"
}